{
  "gene": "UniProtKB:P28566",
  "term_id": "GO:0007198",
  "term_label": "adenylate cyclase-inhibiting serotonin receptor signaling pathway",
  "gene_name": "5-hydroxytryptamine receptor 1E",
  "gene_symbol": "HTR1E"
}